{
  "term_id": "GO:0032434",
  "gene_name": "Desumoylating isopeptidase 1",
  "gene": "UniProtKB:Q6ICB0",
  "term_label": "regulation of proteasomal ubiquitin-dependent protein catabolic process",
  "gene_symbol": "DESI1"
}